{
  "gene_name": "Exosome component 10",
  "term_label": "nuclear exosome (RNase complex)",
  "gene": "UniProtKB:Q01780",
  "gene_symbol": "EXOSC10",
  "term_id": "GO:0000176"
}